{
  "term_label": "structural constituent of chromatin",
  "gene_name": "Histone H3-7",
  "gene": "UniProtKB:Q5TEC6",
  "term_id": "GO:0030527",
  "gene_symbol": "H3-7"
}